urea transport [GO:0015840] (biological process) Relationships: is a type of one-carbon compound transport [GO:0019755]; is a type of GO:0042886 Subtypes: GO:0071918 Sources: GOC:ai, ISBN:0198506732 Definition: The directed movement of urea into, out of or within the cell. Urea is the water-soluble compound H2N-CO-NH2.